{
  "gene_symbol": "FAM177B",
  "gene_name": "Protein FAM177B",
  "term_id": "UNKNOWN:0002",
  "term_label": "Unknown biological process",
  "gene": "UniProtKB:A6PVY3"
}